{
  "gene_symbol": "SLC7A14",
  "term_label": "amino acid transmembrane transporter activity",
  "gene": "UniProtKB:Q8TBB6",
  "term_id": "GO:0015171",
  "gene_name": "Probable cationic amino acid transporter"
}